{
  "term_id": "GO:0042162",
  "gene_name": "CST complex subunit CTC1",
  "gene": "UniProtKB:Q2NKJ3",
  "gene_symbol": "CTC1",
  "term_label": "telomeric DNA binding"
}